{
  "gene_symbol": "HAL",
  "gene": "UniProtKB:P42357",
  "gene_name": "Histidine ammonia-lyase",
  "term_id": "GO:0006548",
  "term_label": "L-histidine catabolic process"
}